{
  "gene_name": "Mitochondrial carnitine_acylcarnitine carrier protein",
  "gene_symbol": "SLC25A20",
  "term_id": "GO:0015227",
  "term_label": "O-acyl-L-carnitine transmembrane transporter activity",
  "gene": "UniProtKB:O43772"
}